U7 snRNA binding [GO:0071209] (molecular function) Note: Note that this term may be useful for annotating other small nuclear RNAs (snRNAs). Relationships: is_a GO:0017069 References: PMID:12975319 Sources: GOC:mah Definition: Binding to a U7 small nuclear RNA (U7 snRNA).